{
  "term_id": "UNKNOWN:0003",
  "gene_name": "5-phosphohydroxy-L-lysine phospho-lyase",
  "gene_symbol": "PHYKPL",
  "term_label": "Unknown cellular component",
  "gene": "UniProtKB:Q8IUZ5"
}